adenylate cyclase-activating G protein-coupled bile acid receptor signaling pathway [GO:0038184] (biological process) Definition: An adenylate cyclase-activating G protein-coupled receptor signaling pathway initiated by a ligand binding to a bile acid receptor on the surface of the target cell, and ending with the regulation of a downstream cellular process. References: PMID:12419312, PMID:19442546, PMID:36409000 Also known as: cell surface bile acid receptor signaling pathway, membrane bile acid receptor signaling pathway Relationships: is a type of cell surface receptor signaling pathway [GO:0007166]; is a type of GO:0007189; is a type of bile acid signaling pathway [GO:0038183]; BFO_0000051 G protein-coupled bile acid receptor activity [GO:0038182]